retrograde axonal transport [GO:0008090] (biological process) Sources: ISBN:0815316194 Relationships: is a type of axonal transport [GO:0098930]; occurs in GO:1904115 Subtypes: GO:0048491, retrograde axonal transport of mitochondrion [GO:0098958], retrograde axonal protein transport [GO:0099642], GO:1990049 Also known as: retrograde axon cargo transport Definition: The directed movement of organelles or molecules along microtubules from the cell periphery toward the cell body in nerve cell axons. Regulation: regulated by regulation of retrograde axon cargo transport [GO:2001017]; RO_0002212 by negative regulation of retrograde axon cargo transport [GO:2001018]; RO_0002213 by positive regulation of retrograde axon cargo transport [GO:2001019]